{
  "gene_symbol": "H2AC21",
  "gene_name": "Histone H2A type 2-B",
  "term_label": "nucleosome",
  "term_id": "GO:0000786",
  "gene": "UniProtKB:Q8IUE6"
}